negative regulation of peripheral B cell anergy [GO:0002918] (biological process) Sources: GOC:add Relationships: is a type of GO:0002659; is a type of negative regulation of B cell anergy [GO:0002671]; is_a negative regulation of B cell mediated immunity [GO:0002713]; is a type of GO:0002917; RO_0002212 peripheral B cell anergy [GO:0002453] Definition: Any process that stops, prevents, or reduces the frequency, rate, or extent of peripheral B cell anergy. Also known as: down regulation of peripheral B cell anergy, down-regulation of peripheral B cell anergy, downregulation of peripheral B cell anergy, inhibition of peripheral B cell anergy